{
  "term_id": "UNKNOWN:0001",
  "gene_name": "Putative postmeiotic segregation increased 2-like protein 3",
  "gene_symbol": "PMS2P3",
  "term_label": "Unknown molecular function",
  "gene": "UniProtKB:Q13401"
}